{
  "gene": "UniProtKB:Q5T0N1",
  "gene_name": "Cilia- and flagella-associated protein 70",
  "term_label": "Unknown molecular function",
  "gene_symbol": "CFAP70",
  "term_id": "UNKNOWN:0001"
}